{
  "term_label": "endoplasmic reticulum membrane",
  "gene_symbol": "SELENON",
  "gene_name": "Selenoprotein N",
  "term_id": "GO:0005789",
  "gene": "UniProtKB:Q9NZV5"
}